negative regulation of integrin activation [GO:0033624] (biological process) Relationships: is a type of negative regulation of protein-containing complex assembly [GO:0031333]; is_a GO:0033623; negatively regulates GO:0033622 Definition: Any process that stops, prevents, or reduces the frequency, rate, or extent of integrin activation. Sources: GOC:add Also known as: negative regulation of integrin complex activation